hydrogenosomal membrane [GO:0046859] (cellular component) Definition: The lipid bilayer surrounding a hydrogenosome. Relationships: is_a bounding membrane of organelle [GO:0098588]; is part of hydrogenosome [GO:0042566] Also known as: hydrogenosome membrane Sources: GOC:ai